{
  "gene": "UniProtKB:P62861",
  "term_id": "GO:0016567",
  "term_label": "protein ubiquitination",
  "gene_symbol": "FAU",
  "gene_name": "Ubiquitin-like FUBI-ribosomal protein eS30 fusion protein"
}